modified amino acid metabolic process [GO:0006575] (biological process) Sources: GOC:ai Subtypes: argininosuccinate metabolic process [GO:0000053], amino-acid betaine metabolic process [GO:0006577], creatine metabolic process [GO:0006600], phosphocreatine metabolic process [GO:0006603], phosphatidylserine metabolic process [GO:0006658], GO:0006749, GO:0006760, GO:0015939, peptidyl-proline hydroxylation to 3-hydroxy-L-proline [GO:0018400], GO:0018401, glyphosate metabolic process [GO:0018920], GO:0019283, GO:0033477, GO:0042219, modified amino acid biosynthetic process [GO:0042398], thyroid hormone metabolic process [GO:0042403], S-adenosylhomocysteine metabolic process [GO:0046498], hypusine metabolic process [GO:0046516], sarcosine metabolic process [GO:1901052], L-dopa metabolic process [GO:1903184] Definition: The chemical reactions and pathways involving compounds derived from amino acids, organic acids containing one or more amino substituents. Relationships: is a type of GO:0008152 Also known as: amino acid derivative metabolic process, cellular amino acid derivative metabolic process, cellular amino acid derivative metabolism, cellular modified amino acid metabolic process, cellular modified amino acid metabolism, modified amino acid metabolism